{
  "gene_name": "Nucleoporin-62 C-terminal-like protein",
  "term_id": "UNKNOWN:0001",
  "gene_symbol": "NUP62CL",
  "gene": "UniProtKB:Q9H1M0",
  "term_label": "Unknown molecular function"
}